regulation of protein monoubiquitination [GO:1902525] (biological process) Definition: Any process that modulates the frequency, rate or extent of protein monoubiquitination. Relationships: is a type of regulation of protein ubiquitination [GO:0031396]; regulates protein monoubiquitination [GO:0006513] References: PMID:21931591 Sources: GOC:TermGenie Subtypes: negative regulation of protein monoubiquitination [GO:1902526], positive regulation of protein monoubiquitination [GO:1902527] Also known as: regulation of protein monoubiquitinylation, regulation of protein monoubiquitylation